chlamydospore formation [GO:0001410] (biological process) Relationships: is a type of asexual sporulation resulting in formation of a cellular spore [GO:0043936]; is a type of cell development [GO:0048468] Definition: The process whose specific outcome is the progression of the chlamydospore over time, from its formation to the mature structure. A chlamydospores is a mitotic (asexual) one-celled spore, produced primarily for survival, not dispersal, originating endogenously and singly within part of a pre-existing cell and possessing an inner secondary and often thickened cell wall. An example of this is found in Candida albicans. References: PMID:14663094 Sources: GOC:mcc, GOC:mtg_sensu, ISBN:085199377X Also known as: chlamydospore development